{
  "term_id": "GO:0007507",
  "gene_name": "Myocyte-specific enhancer factor 2B",
  "gene": "UniProtKB:Q02080",
  "term_label": "heart development",
  "gene_symbol": "MEF2B"
}